{
  "gene_symbol": "DSP",
  "term_id": "GO:0043588",
  "gene": "UniProtKB:P15924",
  "term_label": "skin development",
  "gene_name": "Desmoplakin"
}